{
  "term_label": "cyclooxygenase pathway",
  "term_id": "GO:0019371",
  "gene_symbol": "CTHRC1",
  "gene": "UniProtKB:Q96CG8",
  "gene_name": "Collagen triple helix repeat-containing protein 1"
}